{
  "term_label": "Unknown cellular component",
  "term_id": "UNKNOWN:0003",
  "gene_name": "Zinc finger transcription factor Trps1",
  "gene": "UniProtKB:Q9UHF7",
  "gene_symbol": "TRPS1"
}